{
  "term_label": "kinetochore",
  "gene_name": "G patch domain-containing protein 11",
  "term_id": "GO:0000776",
  "gene": "UniProtKB:Q8N954",
  "gene_symbol": "GPATCH11"
}